{
  "gene_name": "Protein Wnt-16",
  "term_id": "GO:0060070",
  "gene": "UniProtKB:Q9UBV4",
  "term_label": "canonical Wnt signaling pathway",
  "gene_symbol": "WNT16"
}